cell growth mode switching, filamentous to budding [GO:0097321] (biological process) Definition: The process in which a cell switches from growing as a filament (elongated cells attached end-to-end) to growing as a round budding cell. An example of this is observed in Candida albicans. References: PMID:14617167 Sources: GOC:di Relationships: is_a GO:0070784